{
  "gene_name": "Alpha-protein kinase 1",
  "gene_symbol": "ALPK1",
  "term_label": "protein serine/threonine kinase activity",
  "gene": "UniProtKB:Q96QP1",
  "term_id": "GO:0004674"
}